C-C chemokine receptor CCR4 signaling pathway [GO:0038152] (biological process) Definition: The series of molecular signals initiated by a the C-C chemokine type 2 receptor (CCR4) on the surface of a cell binding to one of it's physiological ligands, and ending with the regulation of a downstream cellular process, e.g. transcription. Also known as: C-C chemokine receptor type 4 signaling pathway, chemokine receptor CCR4 signaling pathway Relationships: is a type of GO:0070098 Sources: GOC:nhn, GOC:signaling Subtypes: CCL2-activated CCR4 signaling pathway [GO:0038153]